{
  "term_label": "monoatomic ion transmembrane transport",
  "term_id": "GO:0034220",
  "gene_symbol": "HTR3E",
  "gene_name": "5-hydroxytryptamine receptor 3E",
  "gene": "UniProtKB:A5X5Y0"
}